{
  "term_label": "positive regulation of T-helper 1 type immune response",
  "gene": "UniProtKB:Q9NPF7",
  "gene_name": "Interleukin-23 subunit alpha",
  "term_id": "GO:0002827",
  "gene_symbol": "IL23A"
}